carnitine O-acetyltransferase activity [GO:0004092] (MF) Definition: Catalysis of the reaction: acetyl-CoA + carnitine = (R)-O-acetylcarnitine + CoA. Also known as: carnitine O-acetyltransferase I activity, carnitine O-acetyltransferase II activity, CATC, acetyl-CoA-carnitine O-acetyltransferase activity, acetyl-CoA:carnitine O-acetyltransferase activity, acetylcarnitine transferase activity, carnitine acetyl coenzyme A transferase activity, carnitine acetylase activity, carnitine acetyltransferase activity, carnitine-acetyl-CoA transferase activity Relationships: is a type of GO:0016406; is a type of O-acetyltransferase activity [GO:0016413] Sources: EC:2.3.1.7, RHEA:21136